{
  "gene_name": "Olfactory receptor 10J4",
  "term_label": "detection of chemical stimulus involved in sensory perception of smell",
  "gene": "UniProtKB:P0C629",
  "term_id": "GO:0050911",
  "gene_symbol": "OR10J4"
}